{
  "term_id": "UNKNOWN:0003",
  "gene": "UniProtKB:Q9BXP2",
  "term_label": "Unknown cellular component",
  "gene_name": "Solute carrier family 12 member 9",
  "gene_symbol": "SLC12A9"
}